{
  "gene_name": "Hexokinase-1",
  "gene_symbol": "HK1",
  "term_id": "GO:0019158",
  "gene": "UniProtKB:P19367",
  "term_label": "mannokinase activity"
}